{
  "gene": "UniProtKB:P08590",
  "term_id": "GO:0031674",
  "gene_name": "Myosin light chain 3",
  "gene_symbol": "MYL3",
  "term_label": "I band"
}